{
  "gene_name": "Putative uncharacterized protein encoded by LINC00271",
  "term_id": "UNKNOWN:0001",
  "term_label": "Unknown molecular function",
  "gene_symbol": "AHI1-DT",
  "gene": "UniProtKB:P0C7V0"
}